{
  "term_id": "UNKNOWN:0003",
  "gene": "UniProtKB:Q7Z6I6",
  "gene_name": "Rho GTPase-activating protein 30",
  "gene_symbol": "ARHGAP30",
  "term_label": "Unknown cellular component"
}